{
  "gene": "UniProtKB:Q8NGC6",
  "gene_symbol": "OR4K17",
  "gene_name": "Olfactory receptor 4K17",
  "term_label": "olfactory receptor activity",
  "term_id": "GO:0004984"
}